{
  "term_id": "UNKNOWN:0001",
  "term_label": "Unknown molecular function",
  "gene": "UniProtKB:Q3LI61",
  "gene_symbol": "KRTAP20-2",
  "gene_name": "Keratin-associated protein 20-2"
}